{
  "term_id": "GO:0005980",
  "gene": "UniProtKB:P35573",
  "term_label": "glycogen catabolic process",
  "gene_symbol": "AGL",
  "gene_name": "Glycogen debranching enzyme"
}